striated muscle atrophy [GO:0014891] (biological process) Definition: A process, occurring in striated muscle, that is characterized by a decrease in protein content, fiber diameter, force production and fatigue resistance in response to different conditions such as starvation, aging and disuse. Subtypes: skeletal muscle atrophy [GO:0014732], cardiac muscle atrophy [GO:0014899] Relationships: is a type of striated muscle adaptation [GO:0014888]; is a type of muscle atrophy [GO:0014889] Sources: GOC:mtg_muscle